MUB1-RAD6-UBR2 ubiquitin ligase complex [GO:1990304] (cellular component) Definition: A ubiquitin ligase complex consisting of MUB1, RAD6 and UBR2 components. It ubiquitinates, and targets for destruction, the RPN4 transcription factor, which upregulates the proteasome genes. The binding of MUB1 may position the RPN4 ubiquitylation site proximal to the Ubiquitin-RAD6 thioester and allow the transfer of Ubiquitin from RAD6 to RPN4. One of its components, MUB1, is a short-lived protein ubiquitinated by the UBR2-RAD6 ubiquitin conjugating enzyme. References: PMID:18070918 Sources: GOC:bhm Note: This complex has been identified in Saccharomyces cerevisiae (UniProt symbol P19812) - see PMID:18070918. Relationships: is_a intracellular protein-containing complex [GO:0140535]; is a type of transferase complex [GO:1990234]